epithelial-mesenchymal cell signaling [GO:0060684] (biological process) Definition: Any process that results in the transfer of information from an epithelial cell to a mesenchymal cell where it is interpreted. Relationships: is a type of cell-cell signaling [GO:0007267] Sources: GOC:dph Subtypes: regulation of branching involved in salivary gland morphogenesis by epithelial-mesenchymal signaling [GO:0060683], epithelial-mesenchymal signaling involved in prostate gland development [GO:0060738], epithelial-mesenchymal cell signaling involved in lung development [GO:0061111] Also known as: epithelial-mesenchymal cell signalling